{
  "gene_symbol": "KLRC1",
  "gene": "UniProtKB:P26715",
  "term_id": "GO:0062080",
  "gene_name": "NKG2-A_NKG2-B type II integral membrane protein",
  "term_label": "inhibitory MHC class Ib receptor activity"
}